{
  "term_id": "UNKNOWN:0001",
  "gene_symbol": "C6orf15",
  "term_label": "Unknown molecular function",
  "gene": "UniProtKB:Q6UXA7",
  "gene_name": "Uncharacterized protein C6orf15"
}